{
  "term_label": "Unknown cellular component",
  "term_id": "UNKNOWN:0003",
  "gene": "UniProtKB:A8MUA0",
  "gene_symbol": "A8MUA0",
  "gene_name": "Putative UPF0607 protein ENSP00000381514"
}